symbiont-mediated perturbation of host phytoalexin production [GO:0052165] (biological process) References: PMID:6870275 Sources: GOC:mtg_pamgo_17jul06 Relationships: is a type of symbiont-mediated evasion of host immune response [GO:0042783] Also known as: response to host phytoalexin production, response to phytoalexin production by other organism involved in symbiotic interaction, evasion or tolerance by symbiont of host-produced phytoalexins, evasion or tolerance of phytoalexins, evasion or tolerance of phytoalexins produced by host in response to organism, symbiont defense to host-produced phytoalexin, host phytoalexin detoxification, modulation by organism of phytoalexin production in other organism involved in symbiotic interaction, modulation by symbiont of host phytoalexin production, phytoalexin detoxification Definition: Any process in which a symbiont modulates the frequency, rate or extent of production of phytoalexins as part of the defense response of the host organism. The host is defined as the larger of the organisms involved in a symbiotic interaction. Subtypes: GO:1990217